{
  "gene_name": "Zinc finger HIT domain-containing protein 1",
  "gene": "UniProtKB:O43257",
  "term_id": "UNKNOWN:0002",
  "term_label": "Unknown biological process",
  "gene_symbol": "ZNHIT1"
}